{
  "term_label": "DNA-binding transcription factor activity, RNA polymerase II-specific",
  "gene_name": "Ventral anterior homeobox 2",
  "gene_symbol": "VAX2",
  "gene": "UniProtKB:Q9UIW0",
  "term_id": "GO:0000981"
}